{
  "gene_name": "Peroxisomal membrane protein PMP34",
  "term_label": "FMN transmembrane transporter activity",
  "gene_symbol": "SLC25A17",
  "gene": "UniProtKB:O43808",
  "term_id": "GO:0044610"
}